{
  "gene_name": "Zinc finger protein 347",
  "gene": "UniProtKB:Q96SE7",
  "term_label": "nucleus",
  "gene_symbol": "ZNF347",
  "term_id": "GO:0005634"
}